mannose trimming involved in glycoprotein ERAD pathway [GO:1904382] (biological process) Definition: The removal of one or more alpha 1,2-linked mannose residues from a mannosylated protein that occurs as part of glycoprotein ER-associated glycoprotein degradation (gpERAD). References: PMID:24519966 Sources: GOC:PARL, GOC:TermGenie, GOC:bf, GO_REF:0000060 Also known as: mannose trimming involved in misfolded or incompletely synthesized glycoprotein catabolic process, protein alpha-1,2-demannosylation involved in ER-associated glycoprotein degradation, protein alpha-1,2-demannosylation involved in glycoprotein ERAD, protein alpha-1,2-demannosylation involved in glycoprotein ERAD pathway, protein alpha-1,2-demannosylation involved in gpERAD, glycoprotein mannose trimming involved in ER-associated glycoprotein degradation, glycoprotein mannose trimming involved in glycoprotein ERAD, glycoprotein mannose trimming involved in glycoprotein ERAD pathway, glycoprotein mannose trimming involved in gpERAD Relationships: is a type of protein deglycosylation involved in glycoprotein catabolic process [GO:0035977]; is a type of GO:0036508; is part of ubiquitin-dependent glycoprotein ERAD pathway [GO:0097466]